regulation of innate immune response [GO:0045088] (biological process) Definition: Any process that modulates the frequency, rate or extent of the innate immune response, the organism's first line of defense against infection. Sources: GOC:ebc Relationships: is a type of regulation of response to biotic stimulus [GO:0002831]; is a type of regulation of defense response [GO:0031347]; is a type of regulation of response to external stimulus [GO:0032101]; is a type of regulation of immune response [GO:0050776]; regulates GO:0045087 Subtypes: regulation of complement activation, lectin pathway [GO:0001868], regulation of natural killer cell mediated immunity [GO:0002715], regulation of plant-type hypersensitive response [GO:0010363], regulation of complement activation, alternative pathway [GO:0030451], GO:0035007, positive regulation of innate immune response [GO:0045089], negative regulation of innate immune response [GO:0045824], regulation of respiratory burst involved in inflammatory response [GO:0060264], GO:0060330, GO:0060338, regulation of pattern recognition receptor signaling pathway [GO:0062207], regulation of age-related resistance [GO:1904248], regulation of antifungal innate immune response [GO:1905034], regulation of innate immunity memory response [GO:1905680]